{
  "term_label": "lipid binding",
  "gene": "UniProtKB:O14791",
  "term_id": "GO:0008289",
  "gene_name": "Apolipoprotein L1",
  "gene_symbol": "APOL1"
}